{
  "gene_symbol": "NFE4",
  "term_label": "nucleus",
  "term_id": "GO:0005634",
  "gene_name": "Transcription factor NF-E4",
  "gene": "UniProtKB:Q86UQ8"
}